{
  "term_id": "UNKNOWN:0001",
  "term_label": "Unknown molecular function",
  "gene_symbol": "RASL10A",
  "gene_name": "Ras-like protein family member 10A",
  "gene": "UniProtKB:Q92737"
}